{
  "term_label": "positive regulation of chemokine (C-X-C motif) ligand 2 production",
  "gene": "UniProtKB:P58753",
  "gene_symbol": "TIRAP",
  "term_id": "GO:2000343",
  "gene_name": "Toll_interleukin-1 receptor domain-containing adapter protein"
}